{
  "gene_symbol": "FBXO24",
  "term_id": "UNKNOWN:0001",
  "gene_name": "F-box only protein 24",
  "term_label": "Unknown molecular function",
  "gene": "UniProtKB:O75426"
}